{
  "term_id": "GO:0005681",
  "term_label": "spliceosomal complex",
  "gene": "UniProtKB:A6NEQ0",
  "gene_symbol": "RBMY1E",
  "gene_name": "RNA-binding motif protein, Y chromosome, family 1 member E"
}